{
  "gene": "UniProtKB:O95785",
  "term_id": "GO:0000981",
  "gene_symbol": "WIZ",
  "gene_name": "Protein Wiz",
  "term_label": "DNA-binding transcription factor activity, RNA polymerase II-specific"
}